positive regulation of mesenchymal to epithelial transition involved in metanephros morphogenesis [GO:0072108] (biological process) Relationships: is a type of regulation of mesenchymal to epithelial transition involved in metanephros morphogenesis [GO:0003339]; is a type of positive regulation of morphogenesis of an epithelium [GO:1905332]; is a type of positive regulation of epithelial cell differentiation involved in kidney development [GO:2000698]; RO_0002213 mesenchymal to epithelial transition involved in metanephros morphogenesis [GO:0003337] Definition: Any process that increases the rate, frequency or extent of the transition where a mesenchymal cell establishes apical/basolateral polarity, forms intercellular adhesive junctions, synthesizes basement membrane components and becomes an epithelial cell that will contribute to the shaping of the metanephros. Sources: GOC:mtg_kidney_jan10